{
  "gene_symbol": "FRRS1L",
  "gene": "UniProtKB:Q9P0K9",
  "term_label": "Unknown molecular function",
  "term_id": "UNKNOWN:0001",
  "gene_name": "DOMON domain-containing protein FRRS1L"
}